{
  "gene": "UniProtKB:O00487",
  "term_id": "GO:0005634",
  "gene_name": "26S proteasome non-ATPase regulatory subunit 14",
  "gene_symbol": "PSMD14",
  "term_label": "nucleus"
}